nephron development [GO:0072006] (biological process) Subtypes: GO:0039019, GO:0061215, long nephron development [GO:0072029], GO:0072030, metanephric nephron development [GO:0072210] Sources: GOC:mtg_kidney_jan10 Also known as: nephrogenesis Relationships: is a type of anatomical structure development [GO:0048856]; is part of kidney development [GO:0001822] Definition: The process whose specific outcome is the progression of the nephron over time, from its formation to the mature structure. A nephron is the functional unit of the kidney.